class I DNA-(apurinic or apyrimidinic site) endonuclease activity [GO:0140078] (molecular function) Relationships: is a type of DNA-(apurinic or apyrimidinic site) endonuclease activity [GO:0003906]; is a type of carbon-oxygen lyase activity [GO:0016835] Also known as: AP site-DNA 5'-phosphomonoester-lyase activity, DNA-(apurinic or apyrimidinic site) 5'-phosphomonoester-lyase activity, DNA-(apurinic or apyrimidinic site) lyase activity, class I DNA-(apurinic or apyrimidinic site) lyase activity, AP endonuclease class I activity, AP lyase activity, class I AP endonuclease activity Definition: Catalysis of the cleavage of an AP site 3' of the baseless site by a beta-lyase mechanism, leaving an unsaturated aldehyde, termed a 3'-(4-hydroxy-5-phospho-2-pentenal) residue, and a 5'-phosphate. References: PMID:1698278 Sources: RHEA:66592